mitochondrial tRNA methylation [GO:0070901] (biological process) Relationships: is a type of tRNA methylation [GO:0030488]; is a type of mitochondrial tRNA modification [GO:0070900] Sources: GOC:mah, GOC:mcc Definition: The posttranscriptional addition of methyl groups to specific residues in a mitochondrial tRNA molecule.